voltage-gated calcium channel activity involved in regulation of presynaptic cytosolic calcium levels [GO:0099626] (molecular function) Relationships: is a type of voltage-gated calcium channel activity involved in regulation of cytosolic calcium levels [GO:0099511]; is part of regulation of presynaptic cytosolic calcium ion concentration [GO:0099509]; occurs in presynapse [GO:0098793] References: PMID:15548655 Sources: GOC:dos Also known as: voltage-gated calcium channel activity involved in regulation of presynaptic cytosolic calcium levels Definition: Regulation of presynaptic cytosolic calcium ion concentrations via the action of voltage-gated calcium ion channels.